{
  "gene": "UniProtKB:Q96K21",
  "gene_symbol": "ZFYVE19",
  "term_label": "phosphatidylinositol-3-phosphate binding",
  "gene_name": "Abscission_NoCut checkpoint regulator",
  "term_id": "GO:0032266"
}